positive regulation of muscle adaptation [GO:0014744] (biological process) Also known as: positive regulation of muscle plasticity Sources: GOC:mtg_muscle Relationships: is a type of regulation of muscle adaptation [GO:0043502]; is a type of GO:0048584; is a type of positive regulation of multicellular organismal process [GO:0051240]; RO_0002213 muscle adaptation [GO:0043500] Definition: Any process that activates or increases the frequency, rate or extent of muscle adaptation. Subtypes: GO:0010615, positive regulation of muscle atrophy [GO:0014737], positive regulation of muscle hyperplasia [GO:0014739], positive regulation of skeletal muscle hypertrophy [GO:1904206], positive regulation of smooth muscle hypertrophy [GO:1905149]